{
  "term_id": "GO:0005484",
  "term_label": "SNAP receptor activity",
  "gene": "UniProtKB:Q9UNK0",
  "gene_symbol": "STX8",
  "gene_name": "Syntaxin-8"
}